{
  "term_label": "cytoskeleton",
  "gene_name": "FERM domain-containing protein 3",
  "gene": "UniProtKB:A2A2Y4",
  "gene_symbol": "FRMD3",
  "term_id": "GO:0005856"
}